(1->3)-beta-D-glucan binding [GO:0001872] (molecular function) References: PMID:14707091 Definition: Binding to a (1->3)-beta-D-glucan. Also known as: 1,3-beta-D-glucan binding, callose binding, zymosan binding Relationships: is a type of GO:0030247